{
  "term_id": "GO:0005776",
  "term_label": "autophagosome",
  "gene_symbol": "RAB3GAP2",
  "gene": "UniProtKB:Q9H2M9",
  "gene_name": "Rab3 GTPase-activating protein non-catalytic subunit"
}